{
  "gene_name": "Platelet-activating factor acetylhydrolase IB subunit beta",
  "term_id": "GO:0031023",
  "term_label": "microtubule organizing center organization",
  "gene_symbol": "PAFAH1B1",
  "gene": "UniProtKB:P43034"
}